positive regulation of retinal cell programmed cell death [GO:0046670] (BP) Definition: Any process that activates or increases the frequency, rate or extent of programmed cell death that occurs in the retina. Also known as: positive regulation of retinal programmed cell death, up regulation of retinal programmed cell death, up-regulation of retinal programmed cell death, upregulation of retinal programmed cell death, activation of retinal programmed cell death, stimulation of retinal programmed cell death Sources: GOC:ai, GOC:tb Relationships: is_a GO:0043068; is a type of regulation of retinal cell programmed cell death [GO:0046668]; is a type of positive regulation of developmental process [GO:0051094]; positively regulates retinal cell programmed cell death [GO:0046666] Subtypes: positive regulation of compound eye retinal cell programmed cell death [GO:0046672]